keto-3-deoxy-D-manno-octulosonic acid biosynthetic process [GO:0019294] (biological process) Relationships: is a type of monosaccharide biosynthetic process [GO:0046364]; is a type of carboxylic acid biosynthetic process [GO:0046394]; BFO_0000050 lipopolysaccharide biosynthetic process [GO:0009103] Also known as: KDO biosynthesis, KDO biosynthetic process, keto-3-deoxy-D-manno-octulosonic acid anabolism, keto-3-deoxy-D-manno-octulosonic acid biosynthesis, keto-3-deoxy-D-manno-octulosonic acid formation, keto-3-deoxy-D-manno-octulosonic acid synthesis, ketodeoxyoctanoate biosynthetic process Definition: The chemical reactions and pathways resulting in the formation of keto-3-deoxy-D-manno-octulosonic acid, an acidic sugar present in lipopolysaccharides of the outer membranes of some Gram-negative bacteria. Sources: ISBN:0198506732